calcium:sodium antiporter activity involved in regulation of cardiac muscle cell membrane potential [GO:0086038] (MF) Relationships: is a type of calcium:sodium antiporter activity [GO:0005432]; is part of GO:0086036 Definition: Enables the transfer of a solute or solutes from one side of a membrane to the other according to the reaction: Ca2+(in) + Na+(out) = Ca2+(out) + Na+(in), which contributes to regulating the membrane potential of a cardiac muscle cell. Sources: GOC:BHF, GOC:mtg_cardiac_conduct_nov11